{
  "term_id": "GO:0030368",
  "gene_symbol": "IL17RA",
  "gene": "UniProtKB:Q96F46",
  "term_label": "interleukin-17 receptor activity",
  "gene_name": "Interleukin-17 receptor A"
}